{
  "term_id": "UNKNOWN:0001",
  "gene_symbol": "Q6ZTC4",
  "gene_name": "Putative uncharacterized protein FLJ44790",
  "term_label": "Unknown molecular function",
  "gene": "UniProtKB:Q6ZTC4"
}